imidazoleglycerol-phosphate dehydratase activity [GO:0004424] (molecular function) Definition: Catalysis of the reaction: D-erythro-1-(imidazol-4-yl)glycerol 3-phosphate = 3-(imidazol-4-yl)-2-oxopropyl phosphate + H2O. Sources: EC:4.2.1.19, RHEA:11040 Also known as: imidazoleglycerol phosphate dehydratase activity, D-erythro-1-(imidazol-4-yl)glycerol 3-phosphate hydro-lyase [3-(imidazol-4-yl)-2-oxopropyl-phosphate-forming], D-erythro-1-(imidazol-4-yl)glycerol 3-phosphate hydro-lyase activity, IGP dehydratase activity Relationships: is a type of hydro-lyase activity [GO:0016836]